{
  "gene": "UniProtKB:O76039",
  "gene_symbol": "CDKL5",
  "gene_name": "Cyclin-dependent kinase-like 5",
  "term_label": "Unknown biological process",
  "term_id": "UNKNOWN:0002"
}